{
  "term_id": "GO:2000300",
  "gene": "UniProtKB:Q9UQ26",
  "gene_symbol": "RIMS2",
  "gene_name": "Regulating synaptic membrane exocytosis protein 2",
  "term_label": "regulation of synaptic vesicle exocytosis"
}